{
  "gene_name": "Zinc finger FYVE domain-containing protein 9",
  "term_label": "early endosome membrane",
  "gene": "UniProtKB:O95405",
  "gene_symbol": "ZFYVE9",
  "term_id": "GO:0031901"
}